{
  "term_label": "Unknown biological process",
  "gene_symbol": "A0A087WUM9",
  "term_id": "UNKNOWN:0002",
  "gene_name": "Uncharacterized protein",
  "gene": "UniProtKB:A0A087WUM9"
}